{
  "gene_symbol": "C1R",
  "term_id": "GO:0031638",
  "gene_name": "Complement C1r subcomponent",
  "gene": "UniProtKB:P00736",
  "term_label": "zymogen activation"
}